{
  "gene": "UniProtKB:Q9BR26",
  "gene_symbol": "OCSTAMP",
  "term_label": "Unknown cellular component",
  "term_id": "UNKNOWN:0003",
  "gene_name": "Osteoclast stimulatory transmembrane protein"
}